{
  "gene": "UniProtKB:Q24JP5",
  "term_label": "membrane",
  "term_id": "GO:0016020",
  "gene_name": "Transmembrane protein 132A",
  "gene_symbol": "TMEM132A"
}